{
  "gene_symbol": "MOB1A",
  "gene": "UniProtKB:Q9H8S9",
  "gene_name": "MOB kinase activator 1A",
  "term_id": "GO:0005737",
  "term_label": "cytoplasm"
}